{
  "gene_name": "X antigen family member 5",
  "term_id": "UNKNOWN:0001",
  "term_label": "Unknown molecular function",
  "gene": "UniProtKB:Q8WWM1",
  "gene_symbol": "XAGE5"
}